{
  "gene_symbol": "IGKV2-24",
  "term_id": "GO:0006955",
  "gene": "UniProtKB:A0A0C4DH68",
  "gene_name": "Immunoglobulin kappa variable 2-24",
  "term_label": "immune response"
}